{
  "term_id": "UNKNOWN:0002",
  "gene_name": "Ras-like protein family member 10B",
  "term_label": "Unknown biological process",
  "gene_symbol": "RASL10B",
  "gene": "UniProtKB:Q96S79"
}